{
  "term_label": "cytoplasm",
  "gene_name": "SEC14-like protein 5",
  "term_id": "GO:0005737",
  "gene_symbol": "SEC14L5",
  "gene": "UniProtKB:O43304"
}